{
  "gene_symbol": "SKIDA1",
  "term_id": "UNKNOWN:0003",
  "gene": "UniProtKB:Q1XH10",
  "term_label": "Unknown cellular component",
  "gene_name": "SKI_DACH domain-containing protein 1"
}